{
  "gene": "UniProtKB:P0CJ89",
  "gene_name": "Double homeobox protein 4-like protein 6",
  "gene_symbol": "DUX4L6",
  "term_id": "GO:0006357",
  "term_label": "regulation of transcription by RNA polymerase II"
}